{
  "term_label": "CCR chemokine receptor binding",
  "gene_symbol": "CCL8",
  "gene_name": "C-C motif chemokine 8",
  "gene": "UniProtKB:P80075",
  "term_id": "GO:0048020"
}